{
  "gene_symbol": "SNAPC5",
  "gene": "UniProtKB:O75971",
  "term_label": "Unknown molecular function",
  "term_id": "UNKNOWN:0001",
  "gene_name": "snRNA-activating protein complex subunit 5"
}